{
  "gene_symbol": "RAB2B",
  "term_id": "GO:0005794",
  "term_label": "Golgi apparatus",
  "gene": "UniProtKB:Q8WUD1",
  "gene_name": "Ras-related protein Rab-2B"
}